{
  "gene_name": "Aldehyde dehydrogenase, mitochondrial",
  "term_label": "cellular detoxification of aldehyde",
  "gene_symbol": "ALDH2",
  "term_id": "GO:0110095",
  "gene": "UniProtKB:P05091"
}